pollination [GO:0009856] (biological process) Relationships: is a type of reproductive process [GO:0022414]; is part of GO:0044706 Definition: The cascade of biological processes occurring in plants beginning when the pollen lands on the female reproductive organs of a plant and continuing up to, but not including, fertilization, as defined by sperm-egg cell fusion. References: PMID:10973091 Sources: GOC:tb